regulation of insulin-like growth factor receptor signaling pathway [GO:0043567] (biological process) Definition: Any process that modulates the frequency, rate or extent of insulin-like growth factor receptor signaling. Sources: GOC:bf Also known as: regulation of IGF receptor signaling pathway, regulation of IGF receptor signalling pathway, regulation of insulin-like growth factor receptor signalling pathway Relationships: is a type of GO:0009966; regulates insulin-like growth factor receptor signaling pathway [GO:0048009] Subtypes: GO:0043568, GO:0043569